{
  "term_label": "negative regulation of protein catabolic process",
  "term_id": "GO:0042177",
  "gene": "UniProtKB:O14977",
  "gene_symbol": "AZIN1",
  "gene_name": "Antizyme inhibitor 1"
}